{
  "term_id": "GO:0008380",
  "gene_name": "Protein mago nashi homolog",
  "term_label": "RNA splicing",
  "gene_symbol": "MAGOH",
  "gene": "UniProtKB:P61326"
}